{
  "term_id": "GO:0061844",
  "gene_name": "Lithostathine-1-beta",
  "gene_symbol": "REG1B",
  "gene": "UniProtKB:P48304",
  "term_label": "antimicrobial humoral immune response mediated by antimicrobial peptide"
}